{
  "gene_name": "Transcription factor HES-7",
  "gene": "UniProtKB:Q9BYE0",
  "term_id": "GO:0005634",
  "term_label": "nucleus",
  "gene_symbol": "HES7"
}